iron-sulfur-molybdenum cofactor binding [GO:0044590] (molecular function) Relationships: is_a GO:0051536 References: PMID:18429691 Sources: GOC:mengo_curators, GOC:tt Definition: Binding to iron molybdenum cofactor, the cofactor located at the active site of the molybdenum nitrogenase. Also known as: FeMo co binding, FeMoco binding